conversion of seryl-tRNAsec to selenocys-tRNAsec [GO:0001717] (biological process) Definition: The modification process that results in the conversion of serine, carried by a specialized tRNA(ser) (which can read a UGA anticodon), to selenocysteine. Sources: ISBN:155581073X Relationships: is a type of charged-tRNA amino acid modification [GO:0019988]